{
  "term_label": "SREBP signaling pathway",
  "gene_symbol": "ERLIN2",
  "gene": "UniProtKB:O94905",
  "term_id": "GO:0032933",
  "gene_name": "Erlin-2"
}